{
  "gene_symbol": "EYA2",
  "gene_name": "Eyes absent homolog 2",
  "gene": "UniProtKB:O00167",
  "term_label": "nucleus",
  "term_id": "GO:0005634"
}